{
  "gene": "UniProtKB:O00482",
  "gene_name": "Nuclear receptor subfamily 5 group A member 2",
  "term_id": "GO:0009888",
  "term_label": "tissue development",
  "gene_symbol": "NR5A2"
}